{
  "gene_symbol": "LACRT",
  "gene": "UniProtKB:Q9GZZ8",
  "gene_name": "Extracellular glycoprotein lacritin",
  "term_id": "GO:0005615",
  "term_label": "extracellular space"
}